{
  "term_label": "response to light stimulus",
  "gene_name": "Serotonin N-acetyltransferase",
  "gene": "UniProtKB:Q16613",
  "gene_symbol": "AANAT",
  "term_id": "GO:0009416"
}